positive regulation of AMPA receptor activity [GO:2000969] (biological process) Also known as: positive regulation of alpha-amino-3-hydroxy-5-methyl-4-isoxazole propionate selective glutamate receptor activity Relationships: is a type of GO:0032414; is a type of GO:2000311; positively regulates AMPA glutamate receptor activity [GO:0004971] References: PMID:21423165 Definition: Any process that activates or increases the frequency, rate or extent of AMPA selective glutamate receptor activity.